{
  "gene": "UniProtKB:P05186",
  "gene_symbol": "ALPL",
  "term_label": "bone mineralization",
  "gene_name": "Alkaline phosphatase, tissue-nonspecific isozyme",
  "term_id": "GO:0030282"
}